B cell lineage commitment [GO:0002326] (biological process) Relationships: is_a GO:0045165; is part of B cell differentiation [GO:0030183] Also known as: B lymphocyte lineage commitment, B-cell lineage commitment, B-lymphocyte lineage commitment Sources: GOC:add, ISBN:0781735149 Definition: The process in which a lymphoid progenitor cell becomes committed to become any type of B cell. Subtypes: GO:0002336